{
  "gene_symbol": "CHRNA6",
  "term_label": "presynaptic modulation of chemical synaptic transmission",
  "gene": "UniProtKB:Q15825",
  "term_id": "GO:0099171",
  "gene_name": "Neuronal acetylcholine receptor subunit alpha-6"
}